{
  "term_label": "cholesterol metabolic process",
  "term_id": "GO:0008203",
  "gene_symbol": "CYP11B1",
  "gene": "UniProtKB:P15538",
  "gene_name": "Cytochrome P450 11B1, mitochondrial"
}